{
  "term_label": "Unknown biological process",
  "gene_symbol": "KRTAP10-1",
  "term_id": "UNKNOWN:0002",
  "gene": "UniProtKB:P60331",
  "gene_name": "Keratin-associated protein 10-1"
}